{
  "gene_name": "Complement component C6",
  "gene_symbol": "C6",
  "gene": "UniProtKB:P13671",
  "term_label": "membrane attack complex",
  "term_id": "GO:0005579"
}